{
  "gene_symbol": "SERPINE2",
  "gene_name": "Glia-derived nexin",
  "gene": "UniProtKB:P07093",
  "term_label": "extracellular space",
  "term_id": "GO:0005615"
}